{
  "term_label": "Unknown biological process",
  "gene_name": "Lysosomal protective protein",
  "term_id": "UNKNOWN:0002",
  "gene_symbol": "CTSA",
  "gene": "UniProtKB:P10619"
}